blastocyst hatching [GO:0001835] (biological process) Definition: The hatching of the cellular blastocyst from the zona pellucida. Also known as: blastula hatching Note: See also the Anatomical Dictionary for Mouse Development ontology terms 'TS4, zona pellucida ; EMAP:22' and 'TS5, embryo ; EMAP:23'. Sources: GOC:dph, ISBN:0124020607, ISBN:0198542771 Relationships: is a type of hatching [GO:0035188]; is part of blastocyst development [GO:0001824]